{
  "gene_name": "Dynein axonemal heavy chain 1",
  "term_label": "dynein intermediate chain binding",
  "term_id": "GO:0045505",
  "gene": "UniProtKB:Q9P2D7",
  "gene_symbol": "DNAH1"
}